trehalose-phosphatase activity [GO:0004805] (molecular function) Relationships: is a type of sugar-phosphatase activity [GO:0050308] Sources: EC:3.1.3.12, RHEA:23420 Definition: Catalysis of the reaction: alpha,alpha-trehalose 6-phosphate + H2O = alpha,alpha-trehalose + phosphate. Also known as: trehalose phosphatase activity, trehalose 6-phosphatase activity, trehalose 6-phosphate phosphatase activity, trehalose-6-phosphate phosphohydrolase activity